positive regulation of cellular defense response [GO:0010186] (biological process) Definition: Any process that activates or increases the frequency, rate or extent of cellular defense response. Sources: GOC:sm Relationships: is a type of regulation of cellular defense response [GO:0010185]; is a type of GO:0031349; positively regulates cellular defense response [GO:0006968] Also known as: positive regulation of cellular defence response, up regulation of cellular defense response, up-regulation of cellular defense response, upregulation of cellular defense response, activation of cellular defense response, stimulation of cellular defense response